{
  "term_id": "UNKNOWN:0001",
  "gene_name": "Rho-related GTP-binding protein RhoD",
  "term_label": "Unknown molecular function",
  "gene_symbol": "RHOD",
  "gene": "UniProtKB:O00212"
}